{
  "gene_symbol": "Q8N6K4",
  "gene": "UniProtKB:Q8N6K4",
  "term_label": "Unknown molecular function",
  "gene_name": "Putative uncharacterized protein MGC34800",
  "term_id": "UNKNOWN:0001"
}